positive regulation of ERAD pathway [GO:1904294] (biological process) Relationships: is a type of positive regulation of proteasomal protein catabolic process [GO:1901800]; is a type of regulation of ERAD pathway [GO:1904292]; is a type of GO:1905898; positively regulates GO:0036503 Also known as: positive regulation of endoplasmic reticulum-associated degradation, up regulation of ERAD pathway, up regulation of endoplasmic reticulum-associated degradation, up-regulation of ERAD pathway, up-regulation of endoplasmic reticulum-associated degradation, upregulation of ERAD pathway, upregulation of endoplasmic reticulum-associated degradation, activation of ERAD pathway, activation of endoplasmic reticulum-associated degradation, activation of ER-associated degradation pathway, activation of endoplasmic reticulum-associated protein degradation pathway, positive regulation of ER-associated degradation pathway, positive regulation of endoplasmic reticulum-associated protein degradation pathway, up regulation of ER-associated degradation pathway, up regulation of endoplasmic reticulum-associated protein degradation pathway, up-regulation of ER-associated degradation pathway, up-regulation of endoplasmic reticulum-associated protein degradation pathway, upregulation of ER-associated degradation pathway, upregulation of endoplasmic reticulum-associated protein degradation pathway Definition: Any process that activates or increases the frequency, rate or extent of ERAD pathway. Sources: GOC:PARL, GOC:TermGenie, GOC:bf, GO_REF:0000058